{
  "gene_symbol": "TNFRSF4",
  "gene_name": "Tumor necrosis factor receptor superfamily member 4",
  "gene": "UniProtKB:P43489",
  "term_label": "inflammatory response",
  "term_id": "GO:0006954"
}